{
  "gene_name": "Fez family zinc finger protein 1",
  "gene": "UniProtKB:A0PJY2",
  "term_label": "Unknown cellular component",
  "term_id": "UNKNOWN:0003",
  "gene_symbol": "FEZF1"
}